lactose binding [GO:0030395] (molecular function) Relationships: is a type of disaccharide binding [GO:0048030] Definition: Binding to lactose, a disaccharide of glucose and galactose, the carbohydrate of milk. Sources: GOC:jl, ISBN:0192800981